{
  "gene_symbol": "H2BC9",
  "gene_name": "Histone H2B type 1-H",
  "term_id": "GO:0005615",
  "term_label": "extracellular space",
  "gene": "UniProtKB:Q93079"
}